{
  "gene_symbol": "FJX1",
  "gene_name": "Four-jointed box protein 1",
  "gene": "UniProtKB:Q86VR8",
  "term_label": "protein serine/threonine kinase activity",
  "term_id": "GO:0004674"
}